LDL-containing protein-lipid-RNA complex [GO:1990686] (cellular component) Definition: A protein-lipid-RNA complex containing separate low-density lipoprotein (LDL), lipid and RNA molecules. Separate in this context means not covalently bound to each other. References: PMID:23559634 Sources: GOC:vesicles Note: Examples of LDL-containing protein-lipid-RNA complexes are described in PMID:21423178 and PMID:23559634, both showing evidence that high-density lipoprotein (HDL) and, to a lesser extent, low-density lipoprotein (HDL) transport endogenous microRNAs (miRNAs) and deliver them to recipient cells with functional targeting capabilities. Also see fig. 1 in the review PMID:22028337. Not to be confused with GO:0034362 'low-density lipoprotein particle', which describe complexes of proteins and lipids only, without RNAs. Relationships: is a type of protein-lipid-RNA complex [GO:1990684]